metaphase/anaphase transition of meiotic cell cycle [GO:0044785] (biological process) Relationships: is a type of meiotic cell cycle phase transition [GO:0044771]; is a type of GO:0044784 Definition: The cell cycle process in which a cell progresses from metaphase to anaphase as part of meiosis. Regulation: regulated by GO:1902102; negatively regulated by negative regulation of metaphase/anaphase transition of meiotic cell cycle [GO:1902103]; positively regulated by positive regulation of metaphase/anaphase transition of meiotic cell cycle [GO:1902104] Sources: GOC:mtg_cell_cycle Subtypes: metaphase/anaphase transition of meiosis I [GO:1990949], metaphase/anaphase transition of meiosis II [GO:1990950] Also known as: meiotic metaphase/anaphase transition